{
  "term_label": "Unknown molecular function",
  "term_id": "UNKNOWN:0001",
  "gene_name": "cAMP-responsive element-binding protein-like 2",
  "gene_symbol": "CREBL2",
  "gene": "UniProtKB:O60519"
}